hydroxybutyrate-dimer hydrolase activity [GO:0047989] (molecular function) Definition: Catalysis of the reaction: (R)-3-[(R)-3-hydroxybutanoyloxy]butanoate + H2O = 2 (R)-3-hydroxybutanoate + H+. Sources: EC:3.1.1.22, RHEA:10172 Also known as: (R)-3-((R)-3-hydroxybutanoyloxy)butanoate hydroxybutanoylhydrolase activity, D-(-)-3-hydroxybutyrate-dimer hydrolase activity Relationships: is a type of carboxylic ester hydrolase activity [GO:0052689]